{
  "term_id": "GO:0007283",
  "gene_symbol": "IFT25",
  "gene": "UniProtKB:Q9Y547",
  "gene_name": "Intraflagellar transport protein 25 homolog",
  "term_label": "spermatogenesis"
}